{
  "term_label": "G protein-coupled receptor signaling pathway, coupled to cyclic nucleotide second messenger",
  "gene_name": "Histamine H2 receptor",
  "gene": "UniProtKB:P25021",
  "gene_symbol": "HRH2",
  "term_id": "GO:0007187"
}